{
  "gene": "UniProtKB:Q9NP81",
  "gene_name": "Serine--tRNA ligase, mitochondrial",
  "gene_symbol": "SARS2",
  "term_id": "GO:0005739",
  "term_label": "mitochondrion"
}